leading strand elongation [GO:0006272] (biological process) Sources: GOC:mah, ISBN:071673706X, ISBN:0815316194 Subtypes: GO:1903460 Relationships: is a type of DNA strand elongation involved in DNA replication [GO:0006271]; BFO_0000051 DNA replication, synthesis of primer [GO:0006269]; has part DNA replication, removal of RNA primer [GO:0043137] Definition: The process in which an existing DNA strand is extended continuously in a 5' to 3' direction by activities including the addition of nucleotides to the 3' end of the strand, complementary to an existing template, as part of DNA replication. Leading strand elongation proceeds in the same direction as the replication fork.